{
  "gene_name": "Kelch-like protein 7",
  "gene_symbol": "KLHL7",
  "term_id": "GO:1990756",
  "term_label": "ubiquitin-like ligase-substrate adaptor activity",
  "gene": "UniProtKB:Q8IXQ5"
}